wax biosynthetic process [GO:0010025] (biological process) Definition: The chemical reactions and pathways resulting in the formation of wax, which includes C16 and C18 fatty acids. Also known as: wax anabolism, wax biosynthesis, wax formation, wax synthesis Relationships: is a type of wax metabolic process [GO:0010166]; is a type of GO:1901570 Sources: ISBN:0943088399 Regulation: RO_0002211 by GO:1904276; negatively regulated by negative regulation of wax biosynthetic process [GO:1904277]; positively regulated by positive regulation of wax biosynthetic process [GO:1904278]